{
  "term_id": "GO:0005737",
  "gene_symbol": "PIK3CA",
  "gene": "UniProtKB:P42336",
  "term_label": "cytoplasm",
  "gene_name": "Phosphatidylinositol 4,5-bisphosphate 3-kinase catalytic subunit alpha isoform"
}